{
  "term_label": "Unknown biological process",
  "gene": "UniProtKB:A0A096LNP1",
  "gene_symbol": "DEFB131B",
  "term_id": "UNKNOWN:0002",
  "gene_name": "Beta-defensin 131B"
}